nuclear pore localization [GO:0051664] (biological process) Relationships: is a type of GO:0006997; is a type of GO:0031503; is a type of localization within membrane [GO:0051668] Definition: Any process in which nuclear pores are transported to, or maintained in, a specific location. Sources: GOC:ai Also known as: establishment and maintenance of nuclear pore localization, nuclear pore localisation, nuclear pore distribution, positioning of nuclear pores